positive regulation of metaphase/anaphase transition of cell cycle [GO:1902101] (biological process) Definition: Any process that activates or increases the frequency, rate or extent of metaphase/anaphase transition of cell cycle. Sources: GOC:TermGenie, GOC:mtg_cell_cycle Also known as: up regulation of metaphase/anaphase transition of cell cycle, up-regulation of metaphase/anaphase transition of cell cycle, upregulation of metaphase/anaphase transition of cell cycle, activation of metaphase/anaphase transition of cell cycle Relationships: is_a positive regulation of cell cycle phase transition [GO:1901989]; is a type of regulation of metaphase/anaphase transition of cell cycle [GO:1902099]; positively regulates metaphase/anaphase transition of cell cycle [GO:0044784] Subtypes: positive regulation of mitotic metaphase/anaphase transition [GO:0045842], positive regulation of metaphase/anaphase transition of meiotic cell cycle [GO:1902104]